{
  "gene": "UniProtKB:Q9UGJ0",
  "gene_symbol": "PRKAG2",
  "gene_name": "5'-AMP-activated protein kinase subunit gamma-2",
  "term_label": "AMP binding",
  "term_id": "GO:0016208"
}